{
  "term_label": "positive regulation of BMP signaling pathway",
  "gene": "UniProtKB:Q6ZWJ8",
  "term_id": "GO:0030513",
  "gene_name": "Kielin_chordin-like protein",
  "gene_symbol": "KCP"
}